{
  "gene": "UniProtKB:Q96A58",
  "gene_name": "Ras-related and estrogen-regulated growth inhibitor",
  "term_id": "GO:0007265",
  "term_label": "Ras protein signal transduction",
  "gene_symbol": "RERG"
}